{
  "term_id": "GO:0005783",
  "gene": "UniProtKB:Q8N7C7",
  "gene_name": "RING finger protein 148",
  "term_label": "endoplasmic reticulum",
  "gene_symbol": "RNF148"
}